{
  "term_label": "ciliary basal body",
  "term_id": "GO:0036064",
  "gene": "UniProtKB:Q9BWV7",
  "gene_symbol": "TTLL2",
  "gene_name": "Probable tubulin polyglutamylase TTLL2"
}